positive regulation of caveolin-mediated endocytosis [GO:2001288] (BP) Definition: Any process that activates or increases the frequency, rate or extent of caveolin-mediated endocytosis. Also known as: positive regulation of caveolae-dependent endocytosis, positive regulation of caveolae-mediated endocytosis, positive regulation of caveolin-dependent endocytosis Relationships: is a type of positive regulation of endocytosis [GO:0045807]; is a type of regulation of caveolin-mediated endocytosis [GO:2001286]; positively regulates caveolin-mediated endocytosis [GO:0072584] Sources: GOC:obol